precorrin-6Y C5,15-methyltransferase (decarboxylating) activity [GO:0046025] (molecular function) Also known as: precorrin-6 methyltransferase activity, precorrin-6Y methylase activity, S-adenosyl-L-methionine:1-precorrin-6Y C5,15-methyltransferase (C-12-decarboxylating) Sources: EC:2.1.1.132 Relationships: is a type of S-adenosylmethionine-dependent methyltransferase activity [GO:0008757] Definition: Catalysis of the reaction: 2 S-adenosyl-L-methionine + precorrin-6Y = 2 S-adenosyl-L-homocysteine + precorrin-8X + CO2.